eukaryotic translation initiation factor 3 complex assembly [GO:0070196] (biological process) Relationships: is a type of protein-containing complex assembly [GO:0065003] Also known as: eIF-3 assembly, eIF3 assembly Definition: The aggregation, arrangement and bonding together of a set of components to form the eukaryotic translation initiation factor 3 complex. Sources: GOC:mah